regeneration [GO:0031099] (biological process) Subtypes: somatic embryogenesis [GO:0010262], animal organ regeneration [GO:0031100], neuron projection regeneration [GO:0031102], tissue regeneration [GO:0042246], shoot regeneration [GO:0062210], root regeneration [GO:0062211] Definition: The regrowth of a lost or destroyed body part, such as an organ or tissue. This process may occur via renewal, repair, and/or growth alone (i.e. increase in size or mass). Relationships: is a type of anatomical structure development [GO:0048856] Sources: GOC:mah, GOC:pr